{
  "term_id": "GO:0006491",
  "gene": "UniProtKB:P61647",
  "term_label": "N-glycan processing",
  "gene_name": "Alpha-2,8-sialyltransferase 8F",
  "gene_symbol": "ST8SIA6"
}